{
  "term_id": "UNKNOWN:0001",
  "gene_name": "Vesicle transport protein SFT2C",
  "term_label": "Unknown molecular function",
  "gene_symbol": "SFT2D3",
  "gene": "UniProtKB:Q587I9"
}